{
  "gene_symbol": "ANTXRL",
  "gene_name": "Anthrax toxin receptor-like",
  "term_label": "Unknown biological process",
  "gene": "UniProtKB:A6NF34",
  "term_id": "UNKNOWN:0002"
}